{
  "term_id": "GO:0006357",
  "gene_symbol": "ISX",
  "gene": "UniProtKB:Q2M1V0",
  "term_label": "regulation of transcription by RNA polymerase II",
  "gene_name": "Intestine-specific homeobox"
}